{
  "gene": "UniProtKB:O95076",
  "gene_symbol": "ALX3",
  "term_id": "GO:0000981",
  "term_label": "DNA-binding transcription factor activity, RNA polymerase II-specific",
  "gene_name": "Homeobox protein aristaless-like 3"
}